{
  "term_label": "PAM complex, Tim23 associated import motor",
  "gene_symbol": "GRPEL2",
  "gene_name": "GrpE protein homolog 2, mitochondrial",
  "term_id": "GO:0001405",
  "gene": "UniProtKB:Q8TAA5"
}